{
  "gene_symbol": "TAF7",
  "gene": "UniProtKB:Q15545",
  "term_label": "regulation of transcription by RNA polymerase II",
  "gene_name": "Transcription initiation factor TFIID subunit 7",
  "term_id": "GO:0006357"
}